{
  "term_label": "lipopolysaccharide binding",
  "gene_name": "Beta-defensin 106",
  "term_id": "GO:0001530",
  "gene": "UniProtKB:Q8N104",
  "gene_symbol": "DEFB106A"
}